{
  "term_label": "Unknown biological process",
  "term_id": "UNKNOWN:0002",
  "gene_name": "Large ribosomal subunit protein mL50",
  "gene_symbol": "MRPL50",
  "gene": "UniProtKB:Q8N5N7"
}